{
  "term_label": "Unknown biological process",
  "gene": "UniProtKB:A8MUI8",
  "gene_symbol": "A8MUI8",
  "term_id": "UNKNOWN:0002",
  "gene_name": "Putative UPF0607 protein ENSP00000383783"
}